P-type magnesium transporter activity [GO:0015444] (molecular function) Sources: RHEA:10260 Also known as: magnesium importing ATPase activity, ATP phosphohydrolase (Mg2+-importing), Mg(2+)-importing ATPase activity, Mg2+-importing ATPase activity, magnesium transmembrane transporter activity, phosphorylative mechanism, magnesium-translocating P-type ATPase activity Definition: Enables the transfer of a solute or solutes from one side of a membrane to the other according to the reaction: ATP + H2O + Mg2+(out) = ADP + phosphate + Mg2+(in). Relationships: is a type of magnesium ion transmembrane transporter activity [GO:0015095]; is a type of P-type ion transporter activity [GO:0015662]; is a type of ATPase-coupled monoatomic cation transmembrane transporter activity [GO:0019829]